cellular response to dextromethorphan [GO:1904559] (biological process) Definition: Any process that results in a change in state or activity of a cell (in terms of movement, secretion, enzyme production, gene expression, etc.) as a result of a dextromethorphan stimulus. References: PMID:25796330 Sources: GOC:TermGenie, GOC:mr, GO_REF:0000071 Relationships: is a type of cellular response to isoquinoline alkaloid [GO:0071317]; is a type of cellular response to ether [GO:0071362]; is a type of response to dextromethorphan [GO:1904558]